{
  "term_label": "Unknown molecular function",
  "gene": "UniProtKB:Q8N9W7",
  "gene_name": "Putative transmembrane protein FLJ36131",
  "gene_symbol": "Q8N9W7",
  "term_id": "UNKNOWN:0001"
}